{
  "term_id": "GO:0021952",
  "gene": "UniProtKB:Q96EK5",
  "term_label": "central nervous system projection neuron axonogenesis",
  "gene_symbol": "KIFBP",
  "gene_name": "KIF-binding protein"
}